{
  "term_label": "Unknown molecular function",
  "gene_symbol": "LINC00242",
  "gene_name": "Putative uncharacterized protein encoded by LINC00242",
  "gene": "UniProtKB:Q5T6M2",
  "term_id": "UNKNOWN:0001"
}